{
  "gene_symbol": "MRPS35",
  "gene": "UniProtKB:P82673",
  "gene_name": "Small ribosomal subunit protein mS35",
  "term_id": "GO:0005763",
  "term_label": "mitochondrial small ribosomal subunit"
}